{
  "gene_name": "Translation initiation factor IF-3, mitochondrial",
  "term_label": "translation initiation factor activity",
  "term_id": "GO:0003743",
  "gene_symbol": "MTIF3",
  "gene": "UniProtKB:Q9H2K0"
}